{
  "term_label": "intermediate filament organization",
  "term_id": "GO:0045109",
  "gene_symbol": "KRT7",
  "gene": "UniProtKB:P08729",
  "gene_name": "Keratin, type II cytoskeletal 7"
}